UDP-glucuronate transmembrane transport [GO:0015787] (biological process) Sources: GOC:ai Relationships: is a type of pyrimidine nucleotide-sugar transmembrane transport [GO:0090481]; is a type of GO:1905039 Also known as: UDP-glucuronic acid transmembrane transport, UDP-glucuronic acid transport Definition: The directed movement of UDP-glucuronic acid into, out of or within a cell, or between cells, by means of some agent such as a transporter or pore. UDP-glucuronic acid is a substance composed of glucuronic acid in glycosidic linkage with uridine diphosphate.